MAML3-RBP-Jkappa-ICN2 complex [GO:0071180] (CC) Definition: A protein complex that consists of the intracellular domain of Notch2 (ICN2), the DNA-binding transcription factor RBP-Jkappa, and the transcriptional coactivator Mastermind-like-3 (MAML3); the complex is involved in transcriptional activation in response to Notch-mediated signaling. References: PMID:12370315 Also known as: MAML3-RBP-Jkappa-Notch2 complex Relationships: is a type of nuclear protein-containing complex [GO:0140513]